encapsulation of foreign target [GO:0035010] (BP) Definition: Events resulting in the formation of a multilayered cellular sheath surrounding an invader and thus preventing its development. This defense mechanism is often seen in insects in response to nematodes or parasitoids, which are too large to be phagocytosed by individual hemocytes. In some organisms the capsule is blackened due to melanization. References: PMID:11846478, PMID:12225920 Sources: GOC:bf, GO_REF:0000022 Relationships: is a type of immune effector process [GO:0002252] Subtypes: melanotic encapsulation of foreign target [GO:0035011]